leaf pavement cell development [GO:0090436] (biological process) Relationships: is a type of cell development [GO:0048468]; BFO_0000050 leaf development [GO:0048366] Definition: The process whose specific outcome is the progression of an leaf pavement cell over time, from its formation to the mature structure. Cell development does not include the steps involved in committing a cell to a leaf pavement cell fate. Sources: GOC:tb